{
  "term_label": "regulation of cell cycle phase transition",
  "gene_symbol": "DBF4",
  "term_id": "GO:1901987",
  "gene_name": "Protein DBF4 homolog A",
  "gene": "UniProtKB:Q9UBU7"
}